regulation of chromosome segregation [GO:0051983] (biological process) Relationships: is a type of regulation of cell cycle process [GO:0010564]; regulates chromosome segregation [GO:0007059] Sources: GOC:ai Definition: Any process that modulates the frequency, rate or extent of chromosome segregation, the process in which genetic material, in the form of chromosomes, is organized and then physically separated and apportioned to two or more sets. Subtypes: GO:0033045, GO:0051984, GO:0051985, GO:0060629, regulation of chromosome separation [GO:1905818]